{
  "term_id": "UNKNOWN:0001",
  "gene_symbol": "FBXL19-AS1",
  "term_label": "Unknown molecular function",
  "gene": "UniProtKB:Q494R0",
  "gene_name": "Putative uncharacterized protein FBXL19-AS1"
}